{
  "gene_name": "SH3 domain-binding protein 2",
  "term_label": "Unknown cellular component",
  "term_id": "UNKNOWN:0003",
  "gene": "UniProtKB:P78314",
  "gene_symbol": "SH3BP2"
}